{
  "gene": "UniProtKB:Q9P0B6",
  "gene_name": "Coiled-coil domain-containing protein 167",
  "gene_symbol": "CCDC167",
  "term_id": "UNKNOWN:0001",
  "term_label": "Unknown molecular function"
}